{
  "term_label": "substrate adhesion-dependent cell spreading",
  "gene": "UniProtKB:Q9Y6N6",
  "term_id": "GO:0034446",
  "gene_symbol": "LAMC3",
  "gene_name": "Laminin subunit gamma-3"
}